{
  "term_label": "Unknown molecular function",
  "gene_symbol": "TNXB",
  "gene": "UniProtKB:P22105",
  "term_id": "UNKNOWN:0001",
  "gene_name": "Tenascin-X"
}